mossy fiber rosette [GO:0097471] (cellular component) Definition: A synapse of a mossy fiber onto the dendrite of a granule cell; each mossy fiber can have up to 50 rosettes. Sources: NIF_Subcellular:nlx_subcell_091021, Wikipedia:Mossy_fiber_(cerebellum) Relationships: is a type of asymmetric synapse [GO:0032279] Also known as: cerebellar mossy fiber to granule cell synapse